{
  "term_id": "GO:0034456",
  "term_label": "UTP-C complex",
  "gene": "UniProtKB:Q9H6R4",
  "gene_name": "Nucleolar protein 6",
  "gene_symbol": "NOL6"
}